{
  "gene": "UniProtKB:Q6NZ67",
  "term_id": "UNKNOWN:0001",
  "gene_name": "Mitotic-spindle organizing protein 2B",
  "gene_symbol": "MZT2B",
  "term_label": "Unknown molecular function"
}